{
  "gene_name": "Glutamate receptor ionotropic, NMDA 1",
  "term_id": "GO:0017146",
  "term_label": "NMDA selective glutamate receptor complex",
  "gene": "UniProtKB:Q05586",
  "gene_symbol": "GRIN1"
}